melatonin binding [GO:1904408] (molecular function) References: PMID:10379923 Sources: GOC:TermGenie, GOC:mr, GO_REF:0000067 Definition: Binding to melatonin. Relationships: is a type of amide binding [GO:0033218]